{
  "gene_name": "2-Hydroxyacid oxidase 2",
  "term_id": "UNKNOWN:0002",
  "term_label": "Unknown biological process",
  "gene_symbol": "HAO2",
  "gene": "UniProtKB:Q9NYQ3"
}